ecdysis, chitin-based cuticle [GO:0018990] (BP) Sources: GOC:bf, GOC:mtg_sensu Relationships: is a type of GO:0022404; is part of molting cycle, chitin-based cuticle [GO:0007591] Definition: The shedding of the old chitin-based cuticlar fragments during the molting cycle. An example of this is found in Drosophila melanogaster.